starch utilization system complex [GO:0044570] (cellular component) Relationships: is a type of membrane protein complex [GO:0098796]; BFO_0000050 cell outer membrane [GO:0009279] Definition: A bacterial cell envelope-associated multiprotein system, which binds and degrades starch. Also known as: Sus complex References: PMID:19553672 Sources: GOC:mengo_curators, GOC:tt